{
  "gene": "UniProtKB:P53680",
  "gene_symbol": "AP2S1",
  "term_label": "Unknown molecular function",
  "gene_name": "AP-2 complex subunit sigma",
  "term_id": "UNKNOWN:0001"
}